{
  "gene_symbol": "STON1",
  "gene": "UniProtKB:Q9Y6Q2",
  "term_id": "GO:0072583",
  "term_label": "clathrin-dependent endocytosis",
  "gene_name": "Stonin-1"
}